{
  "term_label": "axoneme",
  "term_id": "GO:0005930",
  "gene": "UniProtKB:Q9P2L0",
  "gene_symbol": "WDR35",
  "gene_name": "WD repeat-containing protein 35"
}